{
  "gene_name": "Ras-related protein Rab-3C",
  "gene": "UniProtKB:Q96E17",
  "term_label": "myosin V binding",
  "term_id": "GO:0031489",
  "gene_symbol": "RAB3C"
}